cellulose biosynthetic process [GO:0030244] (BP) Also known as: cellulose anabolism, cellulose biosynthesis, cellulose formation, cellulose synthesis Sources: GOC:mah, ISBN:0198506732 Relationships: is a type of cellulose metabolic process [GO:0030243]; is a type of beta-glucan biosynthetic process [GO:0051274] Regulation: regulated by regulation of cellulose biosynthetic process [GO:2001006]; negatively regulated by negative regulation of cellulose biosynthetic process [GO:2001007]; positively regulated by positive regulation of cellulose biosynthetic process [GO:2001008] Definition: The chemical reactions and pathways resulting in the formation of cellulose, a linear beta1-4 glucan of molecular mass 50-400 kDa with the pyranose units in the -4C1 conformation. Subtypes: plant-type cell wall cellulose biosynthetic process [GO:0052324], bacterial cellulose biosynthetic process [GO:0090540]